{
  "gene_name": "Dysbindin domain-containing protein 2",
  "gene": "UniProtKB:Q9BQY9",
  "term_id": "GO:0009966",
  "gene_symbol": "DBNDD2",
  "term_label": "regulation of signal transduction"
}